{
  "gene_name": "Olfactory receptor 10C1",
  "gene": "UniProtKB:Q96KK4",
  "term_label": "plasma membrane",
  "term_id": "GO:0005886",
  "gene_symbol": "OR10C1"
}